{
  "term_label": "Unknown biological process",
  "gene_symbol": "SLC37A3",
  "gene_name": "Sugar phosphate exchanger 3",
  "term_id": "UNKNOWN:0002",
  "gene": "UniProtKB:Q8NCC5"
}